{
  "term_label": "regulation of clathrin-dependent endocytosis",
  "term_id": "GO:2000369",
  "gene": "UniProtKB:Q9NSY1",
  "gene_symbol": "BMP2K",
  "gene_name": "BMP-2-inducible protein kinase"
}